{
  "gene_symbol": "METTL15P1",
  "term_id": "GO:0070475",
  "gene": "UniProtKB:P0C7V9",
  "gene_name": "Putative methyltransferase-like protein 15P1",
  "term_label": "rRNA base methylation"
}